{
  "term_id": "GO:0036064",
  "term_label": "ciliary basal body",
  "gene_name": "Stabilizer of axonemal microtubules 2",
  "gene": "UniProtKB:Q658L1",
  "gene_symbol": "SAXO2"
}